{
  "gene": "UniProtKB:P48051",
  "term_id": "UNKNOWN:0001",
  "gene_symbol": "KCNJ6",
  "gene_name": "G protein-activated inward rectifier potassium channel 2",
  "term_label": "Unknown molecular function"
}